regulation of lung goblet cell differentiation [GO:1901249] (biological process) Relationships: is a type of regulation of epithelial cell differentiation [GO:0030856]; regulates lung goblet cell differentiation [GO:0060480] Also known as: regulation of pulmonary goblet cell differentiation Sources: GOC:BHF, GOC:TermGenie Subtypes: negative regulation of lung goblet cell differentiation [GO:1901250], GO:1901251 Definition: Any process that modulates the frequency, rate or extent of lung goblet cell differentiation.